{
  "term_id": "GO:0000122",
  "term_label": "negative regulation of transcription by RNA polymerase II",
  "gene": "UniProtKB:Q5TAB7",
  "gene_name": "Protein ripply2",
  "gene_symbol": "RIPPLY2"
}